{
  "term_label": "signal transduction",
  "gene_symbol": "CNTNAP4",
  "gene_name": "Contactin-associated protein-like 4",
  "gene": "UniProtKB:Q9C0A0",
  "term_id": "GO:0007165"
}